{
  "term_id": "UNKNOWN:0001",
  "term_label": "Unknown molecular function",
  "gene_symbol": "TMEM78",
  "gene_name": "Transmembrane protein 78",
  "gene": "UniProtKB:Q5T7P6"
}